calcium ion import into sarcoplasmic reticulum [GO:1990036] (biological process) References: PMID:17286271 Sources: GOC:BHF Relationships: is a type of intracellular transport [GO:0046907]; is a type of GO:0070296; occurs in cytoplasm [GO:0005737] Definition: The directed movement of calcium ions into a sarcoplasmic reticulum. Regulation: regulated by GO:1902080; RO_0002212 by negative regulation of calcium ion import into sarcoplasmic reticulum [GO:1902081]; positively regulated by positive regulation of calcium ion import into sarcoplasmic reticulum [GO:1902082]